{
  "term_id": "GO:0016604",
  "gene_name": "Polyglutamine-binding protein 1",
  "term_label": "nuclear body",
  "gene_symbol": "PQBP1",
  "gene": "UniProtKB:O60828"
}